valine transport [GO:0015829] (biological process) Also known as: L-valine transport Definition: The directed movement of valine, 2-amino-3-methylbutanoic acid, into, out of or within a cell, or between cells, by means of some agent such as a transporter or pore. Relationships: is_a branched-chain amino acid transport [GO:0015803]; is a type of GO:0015804 Subtypes: GO:1903785 Sources: GOC:ai